{
  "term_label": "Unknown molecular function",
  "term_id": "UNKNOWN:0001",
  "gene": "UniProtKB:Q96F81",
  "gene_symbol": "DISP1",
  "gene_name": "Protein dispatched homolog 1"
}